ADP catabolic process [GO:0046032] (biological process) Relationships: is a type of purine ribonucleotide catabolic process [GO:0009154]; is a type of GO:0009181; is_a ADP metabolic process [GO:0046031] Definition: The chemical reactions and pathways resulting in the breakdown of ADP, adenosine 5'-diphosphate. Sources: GOC:go_curators Subtypes: glycolytic process [GO:0006096] Also known as: ADP breakdown, ADP catabolism, ADP degradation